detection of monosaccharide stimulus [GO:0034287] (biological process) Relationships: is a type of detection of carbohydrate stimulus [GO:0009730]; is a type of response to monosaccharide [GO:0034284] Definition: The series of events in which a stimulus from a monosaccharide is received and converted into a molecular signal. Sources: GOC:mah Subtypes: detection of hexose stimulus [GO:0009732] Also known as: perception of monosaccharide stimulus